{
  "term_id": "GO:0003677",
  "gene": "UniProtKB:Q5T6S3",
  "gene_name": "PHD finger protein 19",
  "term_label": "DNA binding",
  "gene_symbol": "PHF19"
}